{
  "term_id": "GO:0005634",
  "term_label": "nucleus",
  "gene_name": "F-box_WD repeat-containing protein 7",
  "gene_symbol": "FBXW7",
  "gene": "UniProtKB:Q969H0"
}